cellular response to neutral pH [GO:0036244] (biological process) Definition: Any process that results in a change in state or activity of a cell (in terms of movement, secretion, enzyme production, gene expression, etc.) as a result of a neutral pH (pH close to 7) stimulus. pH is a measure of the acidity or basicity of an aqueous solution. Sources: GOC:di, Wikipedia:PH Relationships: is a type of response to neutral pH [GO:0036176]; is_a GO:0071467